{
  "term_label": "gonadotropin-releasing hormone receptor activity",
  "term_id": "GO:0004968",
  "gene_symbol": "GNRHR2",
  "gene_name": "Putative gonadotropin-releasing hormone II receptor",
  "gene": "UniProtKB:Q96P88"
}